positive regulation of sister chromatid cohesion [GO:0045876] (biological process) Also known as: up regulation of sister chromatid cohesion, up-regulation of sister chromatid cohesion, upregulation of sister chromatid cohesion, activation of sister chromatid cohesion, stimulation of sister chromatid cohesion Sources: GOC:go_curators Definition: Any process that activates or increases the frequency, rate or extent of sister chromatid cohesion. Relationships: is a type of GO:0007063; is a type of positive regulation of cell cycle process [GO:0090068]; is a type of positive regulation of chromosome organization [GO:2001252]; positively regulates sister chromatid cohesion [GO:0007062] Subtypes: positive regulation of maintenance of sister chromatid cohesion [GO:0034093]